regulation of cellular response to drug [GO:2001038] (biological process) Relationships: is a type of regulation of cellular process [GO:0050794]; is a type of regulation of response to drug [GO:2001023]; RO_0002211 GO:0071466 Subtypes: negative regulation of cellular response to drug [GO:2001039], positive regulation of cellular response to drug [GO:2001040] Definition: Any process that modulates the frequency, rate or extent of cellular response to drug. Sources: GOC:obol